{
  "term_label": "postsynaptic density membrane",
  "term_id": "GO:0098839",
  "gene": "UniProtKB:Q13224",
  "gene_name": "Glutamate receptor ionotropic, NMDA 2B",
  "gene_symbol": "GRIN2B"
}